nitric oxide catabolic process [GO:0046210] (biological process) Definition: The chemical reactions and pathways resulting in the breakdown of nitric oxide, nitrogen monoxide (NO), a colorless gas only slightly soluble in water. Also known as: nitric oxide breakdown, nitric oxide catabolism, nitric oxide degradation Relationships: is a type of catabolic process [GO:0009056]; is_a nitric oxide metabolic process [GO:0046209] Sources: GOC:ai